{
  "gene_symbol": "CPOX",
  "term_label": "protoporphyrinogen IX biosynthetic process",
  "gene_name": "Oxygen-dependent coproporphyrinogen-III oxidase, mitochondrial",
  "gene": "UniProtKB:P36551",
  "term_id": "GO:0006782"
}